{
  "gene_name": "LIM domain transcription factor LMO4",
  "term_label": "nucleus",
  "gene": "UniProtKB:P61968",
  "term_id": "GO:0005634",
  "gene_symbol": "LMO4"
}